pyrimidine deoxyribonucleoside monophosphate catabolic process [GO:0009178] (biological process) Subtypes: dCMP catabolic process [GO:0006249], dTMP catabolic process [GO:0046074], dUMP catabolic process [GO:0046079] Relationships: is a type of pyrimidine nucleoside monophosphate catabolic process [GO:0009131]; is_a deoxyribonucleoside monophosphate catabolic process [GO:0009159]; is a type of pyrimidine deoxyribonucleoside monophosphate metabolic process [GO:0009176] Also known as: pyrimidine deoxyribonucleoside monophosphate breakdown, pyrimidine deoxyribonucleoside monophosphate catabolism, pyrimidine deoxyribonucleoside monophosphate degradation Sources: GOC:go_curators, ISBN:0198506732 Definition: The chemical reactions and pathways resulting in the breakdown of pyrimidine deoxynucleoside monophosphate, a compound consisting of a pyrimidine base linked to a deoxyribose sugar esterified with phosphate on the sugar.